{
  "term_label": "thymocyte migration",
  "gene": "UniProtKB:P51684",
  "term_id": "GO:0072679",
  "gene_symbol": "CCR6",
  "gene_name": "C-C chemokine receptor type 6"
}